{
  "gene_name": "Hexokinase-2",
  "term_label": "mitochondrion",
  "gene": "UniProtKB:P52789",
  "term_id": "GO:0005739",
  "gene_symbol": "HK2"
}